estradiol binding [GO:1903924] (molecular function) References: PMID:9048584 Sources: GOC:TermGenie, GO_REF:0000067 Relationships: is a type of steroid binding [GO:0005496] Definition: Binding to estradiol.